{
  "gene": "UniProtKB:Q6ZTW0",
  "term_id": "GO:0008017",
  "gene_symbol": "TPGS1",
  "gene_name": "Tubulin polyglutamylase complex subunit 1",
  "term_label": "microtubule binding"
}